peroxisomal-mitochondrial contact site [GO:0160189] (cellular component) References: PMID:29684109, PMID:38669296 Also known as: PerMit contact, PerMit contact site Definition: An organelle membrane contact site between peroxisomal membrane and mitochondrial outer membrane. Relationships: is a type of GO:0044232